2-oxopent-4-enoate hydratase activity [GO:0008684] (molecular function) Relationships: is a type of hydro-lyase activity [GO:0016836] Also known as: 2-keto-4-pentenoate (vinylpyruvate)hydratase activity, 2-keto-4-pentenoate hydratase activity, 4-hydroxy-2-oxopentanoate hydro-lyase (2-oxopent-4-enoate-forming), 4-hydroxy-2-oxopentanoate hydro-lyase activity, OEH activity Sources: EC:4.2.1.80 Definition: Catalysis of the reaction: 4-hydroxy-2-oxopentanoate = 2-oxopent-4-enoate + H2O.